{
  "term_label": "BMP signaling pathway",
  "gene_name": "Bone morphogenetic protein 8A",
  "term_id": "GO:0030509",
  "gene": "UniProtKB:Q7Z5Y6",
  "gene_symbol": "BMP8A"
}